{
  "term_id": "GO:0050839",
  "gene_name": "Protocadherin gamma-A10",
  "gene": "UniProtKB:Q9Y5H3",
  "term_label": "cell adhesion molecule binding",
  "gene_symbol": "PCDHGA10"
}